{
  "gene": "UniProtKB:Q8IYN0",
  "term_label": "Unknown cellular component",
  "term_id": "UNKNOWN:0003",
  "gene_name": "Zinc finger protein 100",
  "gene_symbol": "ZNF100"
}